{
  "gene": "UniProtKB:P07438",
  "gene_symbol": "MT1B",
  "term_label": "metal ion binding",
  "gene_name": "Metallothionein-1B",
  "term_id": "GO:0046872"
}